D-leucine biosynthetic process [GO:1900833] (biological process) Definition: The chemical reactions and pathways resulting in the formation of D-leucine. References: PMID:10918062 Sources: GOC:TermGenie Also known as: D-leucine anabolism, D-leucine biosynthesis, D-leucine formation, D-leucine synthesis Relationships: is a type of branched-chain amino acid biosynthetic process [GO:0009082]; is a type of GO:0046437